{
  "gene_name": "Transmembrane protein 180",
  "gene": "UniProtKB:Q14CX5",
  "gene_symbol": "MFSD13A",
  "term_label": "Unknown biological process",
  "term_id": "UNKNOWN:0002"
}